{
  "gene": "UniProtKB:A0A1W2PQF6",
  "gene_name": "Immunoglobulin subtype domain-containing protein",
  "term_label": "immune receptor activity",
  "term_id": "GO:0140375",
  "gene_symbol": "A0A1W2PQF6"
}